{
  "term_id": "UNKNOWN:0002",
  "gene_symbol": "NFKBIE",
  "gene": "UniProtKB:O00221",
  "term_label": "Unknown biological process",
  "gene_name": "NF-kappa-B inhibitor epsilon"
}